{
  "term_id": "GO:0019730",
  "gene_name": "Putative cystatin-9-like protein CST9LP1",
  "term_label": "antimicrobial humoral response",
  "gene": "UniProtKB:Q5W188",
  "gene_symbol": "CST9LP1"
}